{
  "term_id": "GO:0005737",
  "term_label": "cytoplasm",
  "gene": "UniProtKB:Q9P2K9",
  "gene_name": "Protein dispatched homolog 3",
  "gene_symbol": "DISP3"
}